{
  "gene_name": "Tubulin beta-6 chain",
  "term_label": "structural constituent of cytoskeleton",
  "term_id": "GO:0005200",
  "gene": "UniProtKB:Q9BUF5",
  "gene_symbol": "TUBB6"
}